phosphatidylserine acyl-chain remodeling [GO:0036150] (biological process) Definition: Remodeling the acyl chains of phosphatidylserine, through sequential deacylation and re-acylation reactions, to generate phosphatidylserine containing different types of fatty acid acyl chains. Relationships: is a type of GO:0006658 References: PMID:18287005, PMID:18458083 Sources: GOC:mw Also known as: phosphatidyl-L-serine acyl-chain remodeling, phosphatidylserine acyl-chain remodelling